{
  "term_label": "cytoplasm",
  "gene_symbol": "PRAMEF1",
  "gene_name": "PRAME family member 1",
  "term_id": "GO:0005737",
  "gene": "UniProtKB:O95521"
}